{
  "gene": "UniProtKB:P04233",
  "gene_symbol": "CD74",
  "term_id": "GO:0060907",
  "term_label": "positive regulation of macrophage cytokine production",
  "gene_name": "HLA class II histocompatibility antigen gamma chain"
}